renin secretion into blood stream [GO:0002001] (BP) Also known as: renin release into blood stream Sources: ISBN:0721643949 Definition: The regulated release of renin into the blood stream by juxtoglomerular cells. Relationships: is a type of protein secretion [GO:0009306]; is a type of GO:0023061; is part of renal response to blood flow involved in circulatory renin-angiotensin regulation of systemic arterial blood pressure [GO:0001999] Regulation: regulated by regulation of renin secretion into blood stream [GO:1900133]; negatively regulated by GO:1900134; positively regulated by positive regulation of renin secretion into blood stream [GO:1900135]